{
  "gene_name": "Serine_threonine-protein kinase Nek1",
  "gene_symbol": "NEK1",
  "term_label": "protein kinase activity",
  "gene": "UniProtKB:Q96PY6",
  "term_id": "GO:0004672"
}